{
  "term_id": "GO:0005634",
  "gene_name": "Heterogeneous nuclear ribonucleoprotein L",
  "gene": "UniProtKB:P14866",
  "gene_symbol": "HNRNPL",
  "term_label": "nucleus"
}